{
  "gene": "UniProtKB:Q9HC52",
  "term_label": "PRC1 complex",
  "term_id": "GO:0035102",
  "gene_name": "Chromobox protein homolog 8",
  "gene_symbol": "CBX8"
}